{
  "gene": "UniProtKB:Q96R67",
  "term_id": "GO:0005886",
  "gene_symbol": "OR4C12",
  "term_label": "plasma membrane",
  "gene_name": "Olfactory receptor 4C12"
}